{
  "gene": "UniProtKB:Q9HAF1",
  "gene_name": "Chromatin modification-related protein MEAF6",
  "term_id": "GO:0035267",
  "term_label": "NuA4 histone acetyltransferase complex",
  "gene_symbol": "MEAF6"
}